{
  "term_label": "extracellular space",
  "gene_symbol": "SERPINB13",
  "gene": "UniProtKB:Q9UIV8",
  "gene_name": "Serpin B13",
  "term_id": "GO:0005615"
}